chordate pharynx development [GO:0160093] (biological process) References: PMID:23020903 Relationships: is a type of pharynx development [GO:0060465] Definition: The process whose specific outcome is the progression of cordate pharynx over time, from its formation to the mature structure.